{
  "term_label": "Unknown molecular function",
  "gene_symbol": "FRY",
  "term_id": "UNKNOWN:0001",
  "gene": "UniProtKB:Q5TBA9",
  "gene_name": "Protein furry homolog"
}